{
  "gene_name": "T cell receptor beta joining 2-3",
  "gene": "UniProtKB:A0A0B4J200",
  "gene_symbol": "TRBJ2-3",
  "term_id": "UNKNOWN:0001",
  "term_label": "Unknown molecular function"
}